regulation of pancreatic amylase secretion [GO:1902276] (biological process) Subtypes: negative regulation of pancreatic amylase secretion [GO:1902277], positive regulation of pancreatic amylase secretion [GO:1902278] Definition: Any process that modulates the frequency, rate or extent of pancreatic amylase secretion. Sources: GOC:TermGenie, GOC:jc Relationships: is a type of regulation of protein secretion [GO:0050708]; regulates pancreatic amylase secretion [GO:0036395]